{
  "gene_symbol": "OR5B3",
  "term_id": "GO:0007186",
  "gene_name": "Olfactory receptor 5B3",
  "gene": "UniProtKB:Q8NH48",
  "term_label": "G protein-coupled receptor signaling pathway"
}